neuromedin K receptor binding [GO:0031836] (molecular function) Sources: GOC:mah, GOC:nln Definition: Binding to a neuromedin K receptor. Relationships: is a type of neurokinin receptor binding [GO:0031834] Also known as: neurokinin-B receptor binding, neuromedin K receptor ligand